positive regulation of deoxyribonuclease activity [GO:0032077] (biological process) Definition: Any process that activates or increases the frequency, rate or extent of deoxyribonuclease activity, the hydrolysis of ester linkages within deoxyribonucleic acid. Sources: GOC:mah Also known as: up regulation of deoxyribonuclease activity, up-regulation of deoxyribonuclease activity, upregulation of deoxyribonuclease activity, activation of deoxyribonuclease activity, stimulation of deoxyribonuclease activity, DNase activator, deoxyribonuclease activator Relationships: is a type of positive regulation of catalytic activity [GO:0043085]; is a type of positive regulation of DNA metabolic process [GO:0051054]; positively regulates GO:0004536 Subtypes: positive regulation of endodeoxyribonuclease activity [GO:0032079]